dCMP metabolic process [GO:0046063] (biological process) Relationships: is a type of GO:0009176; is a type of GO:0009219 Subtypes: GO:0006249, dCMP biosynthetic process [GO:0046064] Definition: The chemical reactions and pathways involving dCMP, deoxycytidine monophosphate. Also known as: dCMP metabolism Sources: GOC:go_curators